{
  "gene_symbol": "PTK2B",
  "gene_name": "Protein-tyrosine kinase 2-beta",
  "term_label": "plasma membrane",
  "term_id": "GO:0005886",
  "gene": "UniProtKB:Q14289"
}